{
  "gene_name": "Phosphoinositide-interacting protein",
  "gene_symbol": "PIRT",
  "gene": "UniProtKB:P0C851",
  "term_label": "transmembrane transporter binding",
  "term_id": "GO:0044325"
}